basic amino acid transport [GO:0015802] (biological process) Sources: GOC:ai Definition: The directed movement of basic amino acids, amino acids with a pH above 7, into, out of or within a cell, or between cells, by means of some agent such as a transporter or pore. Relationships: is a type of amino acid transport [GO:0006865] Subtypes: GO:0015817, lysine transport [GO:0015819], GO:1902024, basic amino acid transmembrane transport [GO:1990822]